response to tumor cell [GO:0002347] (biological process) References: PMID:16730260 Sources: GOC:add, ISBN:0781735149 Relationships: is a type of response to biotic stimulus [GO:0009607] Regulation: regulated by regulation of response to tumor cell [GO:0002834]; negatively regulated by GO:0002835; positively regulated by positive regulation of response to tumor cell [GO:0002836] Definition: Any process that results in a change in state or activity of a cell or an organism (in terms of movement, secretion, enzyme production, gene expression, etc.) as a result of a stimulus from a tumor cell. Subtypes: detection of tumor cell [GO:0002355], defense response to tumor cell [GO:0002357], GO:0002418, cellular response to tumor cell [GO:0071228]